{
  "term_label": "extracellular space",
  "gene": "UniProtKB:Q8IXL6",
  "gene_name": "Extracellular serine_threonine protein kinase FAM20C",
  "gene_symbol": "FAM20C",
  "term_id": "GO:0005615"
}